{
  "gene": "UniProtKB:Q9NSV4",
  "gene_name": "Protein diaphanous homolog 3",
  "term_label": "actin filament",
  "gene_symbol": "DIAPH3",
  "term_id": "GO:0005884"
}